{
  "gene": "UniProtKB:O75317",
  "term_label": "cytosol",
  "gene_name": "Ubiquitin carboxyl-terminal hydrolase 12",
  "gene_symbol": "USP12",
  "term_id": "GO:0005829"
}